mitochondrial methionyl-tRNA aminoacylation [GO:0070155] (BP) Relationships: is a type of methionyl-tRNA aminoacylation [GO:0006431]; is a type of tRNA aminoacylation for mitochondrial protein translation [GO:0070127] Sources: GOC:mah, GOC:mcc Definition: The process of coupling methionine to methionyl-tRNA in a mitochondrion, catalyzed by methionyl-tRNA synthetase. In tRNA aminoacylation, the amino acid is first activated by linkage to AMP and then transferred to either the 2'- or the 3'-hydroxyl group of the 3'-adenosine residue of the tRNA.